calcineurin-mediated signaling [GO:0097720] (biological process) Also known as: calcineurin-mediated signalling, calcineurin signaling Relationships: is a type of calcium-mediated signaling [GO:0019722] Regulation: regulated by regulation of calcineurin-mediated signaling [GO:0106056]; negatively regulated by negative regulation of calcineurin-mediated signaling [GO:0106057]; RO_0002213 by positive regulation of calcineurin-mediated signaling [GO:0106058] References: PMID:25655284, PMID:25878052, PMID:26851544 Sources: GOC:di Definition: Any intracellular signal transduction in which the signal is passed on within the cell by activation of a transcription factor as a consequence of dephosphorylation by Ca(2+)-activated calcineurin. The process begins with calcium-dependent activation of the phosphatase calcineurin. Calcineurin is a calcium- and calmodulin-dependent serine/threonine protein phosphatase with a conserved function in eukaryotic species from yeast to humans. In yeast and fungi, calcineurin regulates stress signaling and cell cycle, and sporulation and virulence in pathogenic fungi. In metazoans, calcineurin is involved in cell commitment, organogenesis and organ development and immune function of T-lymphocytes. By a conserved mechanism, calcineurin phosphatase activates fungal Crz1 and mammalian NFATc by dephosphorylation and translocation of these transcription factors to the nucleus to regulate gene expression. Subtypes: GO:0033173